{
  "gene_name": "Lysophospholipid acyltransferase 1",
  "term_id": "GO:0016020",
  "term_label": "membrane",
  "gene_symbol": "MBOAT1",
  "gene": "UniProtKB:Q6ZNC8"
}